{
  "term_label": "Unknown biological process",
  "term_id": "UNKNOWN:0002",
  "gene": "UniProtKB:Q7Z6W1",
  "gene_name": "Transmembrane and coiled-coil domain-containing protein 2",
  "gene_symbol": "TMCO2"
}